regulation of assembly of large subunit precursor of preribosome [GO:1902627] (biological process) Definition: Any process that modulates the frequency, rate or extent of assembly of a large subunit precursor of preribosome. References: PMID:22735702 Sources: GOC:TermGenie, GOC:di, GO_REF:0000058 Also known as: regulation of preribosome, large subunit precursor formation, regulation of 66S preribosome assembly, regulation of 66S preribosome formation Relationships: is a type of regulation of protein-containing complex assembly [GO:0043254]; regulates assembly of large subunit precursor of preribosome [GO:1902626] Subtypes: positive regulation of assembly of large subunit precursor of preribosome [GO:1902628]